{
  "gene_name": "Cyclin-dependent kinase 15",
  "gene": "UniProtKB:Q96Q40",
  "term_id": "GO:0005634",
  "gene_symbol": "CDK15",
  "term_label": "nucleus"
}